{
  "gene_name": "Claudin-34",
  "gene": "UniProtKB:H7C241",
  "term_label": "Unknown molecular function",
  "term_id": "UNKNOWN:0001",
  "gene_symbol": "CLDN34"
}